{
  "term_label": "DNA-binding transcription repressor activity, RNA polymerase II-specific",
  "gene": "UniProtKB:Q13127",
  "term_id": "GO:0001227",
  "gene_symbol": "REST",
  "gene_name": "RE1-silencing transcription factor"
}